distributive segregation [GO:0032837] (biological process) Relationships: is a type of meiotic chromosome segregation [GO:0045132] Definition: The cell cycle process in which genetic material, in the form of chromosomes, is organized and then physically separated and apportioned to two or more sets during a normally chiasmate meiosis under the condition that chiasma have not occurred between a particular pair of homologs. Distributive segregation is a backup mechanism to ensure the segregation of homologs that have failed to cross over - either as a consequence of mutation or not, as, for example, the 4th chromosome of Drosophila melanogaster (which never exchanges, presumably due to its small size) - but nevertheless segregate normally. Sources: GOC:expert_rsh, GOC:ma, GOC:sart